{
  "gene_name": "Scavenger receptor class F member 1",
  "term_id": "GO:0030169",
  "gene": "UniProtKB:Q14162",
  "term_label": "low-density lipoprotein particle binding",
  "gene_symbol": "SCARF1"
}